response to morphine [GO:0043278] (biological process) Definition: Any process that results in a change in state or activity of a cell or an organism (in terms of movement, secretion, enzyme production, gene expression, etc.) as a result of a morphine stimulus. Morphine is an opioid alkaloid, isolated from opium, with a complex ring structure. Subtypes: cellular response to morphine [GO:0071315] Sources: GOC:ef, GOC:jl Relationships: is a type of response to isoquinoline alkaloid [GO:0014072]